{
  "gene_name": "Late cornified envelope protein 1B",
  "gene": "UniProtKB:Q5T7P3",
  "gene_symbol": "LCE1B",
  "term_id": "UNKNOWN:0002",
  "term_label": "Unknown biological process"
}